{
  "gene": "UniProtKB:P82914",
  "gene_name": "Small ribosomal subunit protein uS15m",
  "gene_symbol": "MRPS15",
  "term_label": "Unknown molecular function",
  "term_id": "UNKNOWN:0001"
}